{
  "gene_name": "GRB10-interacting GYF protein 1",
  "term_label": "cytosol",
  "gene": "UniProtKB:O75420",
  "gene_symbol": "GIGYF1",
  "term_id": "GO:0005829"
}